{
  "term_id": "GO:0071294",
  "gene": "UniProtKB:Q8N339",
  "gene_symbol": "MT1M",
  "gene_name": "Metallothionein-1M",
  "term_label": "cellular response to zinc ion"
}